{
  "gene": "UniProtKB:O75475",
  "gene_symbol": "PSIP1",
  "term_id": "UNKNOWN:0001",
  "term_label": "Unknown molecular function",
  "gene_name": "PC4 and SFRS1-interacting protein"
}